{
  "gene": "UniProtKB:Q8NGG2",
  "term_id": "GO:0007608",
  "gene_symbol": "OR5T2",
  "gene_name": "Olfactory receptor 5T2",
  "term_label": "sensory perception of smell"
}